{
  "term_id": "GO:0007015",
  "gene": "UniProtKB:Q0VAK6",
  "term_label": "actin filament organization",
  "gene_symbol": "LMOD3",
  "gene_name": "Leiomodin-3"
}